{
  "gene_symbol": "EEIG2",
  "term_id": "UNKNOWN:0002",
  "gene_name": "EEIG family member 2",
  "term_label": "Unknown biological process",
  "gene": "UniProtKB:Q5T8I3"
}